{
  "term_id": "GO:0007165",
  "gene_name": "Calcium_calmodulin-dependent protein kinase type 1D",
  "term_label": "signal transduction",
  "gene_symbol": "CAMK1D",
  "gene": "UniProtKB:Q8IU85"
}